{
  "gene_symbol": "IL11",
  "gene": "UniProtKB:P20809",
  "term_label": "positive regulation of MAPK cascade",
  "gene_name": "Interleukin-11",
  "term_id": "GO:0043410"
}